taurine transmembrane transporter activity [GO:0005368] (molecular function) Sources: GOC:ai Definition: Enables the transfer of taurine from one side of a membrane to the other. Taurine (2-aminoethanesulfonic acid) is a sulphur-containing amino acid derivative which is important in the metabolism of fats. Subtypes: GO:0005369, GO:0015411 Relationships: is a type of GO:1901682; BFO_0000050 taurine transmembrane transport [GO:0015734]